uroporphyrinogen III biosynthetic process [GO:0006780] (biological process) Also known as: uroporphyrinogen III anabolism, uroporphyrinogen III biosynthesis, uroporphyrinogen III formation, uroporphyrinogen III synthesis Sources: GOC:ai Definition: The chemical reactions and pathways resulting in the formation of uroporphyrinogen III. Relationships: is a type of porphyrin-containing compound biosynthetic process [GO:0006779]; is a type of carboxylic acid biosynthetic process [GO:0046394]; is a type of uroporphyrinogen III metabolic process [GO:0046502]